{
  "term_id": "GO:0001669",
  "gene_symbol": "LYZL4",
  "gene_name": "Lysozyme-like protein 4",
  "gene": "UniProtKB:Q96KX0",
  "term_label": "acrosomal vesicle"
}